{
  "gene_symbol": "IL2",
  "gene_name": "Interleukin-2",
  "gene": "UniProtKB:P60568",
  "term_id": "GO:0005125",
  "term_label": "cytokine activity"
}